{
  "gene": "UniProtKB:Q8NGF4",
  "term_id": "GO:0005549",
  "gene_symbol": "OR5AP2",
  "gene_name": "Olfactory receptor 5AP2",
  "term_label": "odorant binding"
}